neuromuscular process [GO:0050905] (biological process) Subtypes: startle response [GO:0001964], musculoskeletal movement [GO:0050881], GO:0050884, GO:0050885 Also known as: neuromotor process, neuromuscular physiological process Relationships: is a type of GO:0050877 Sources: GOC:ai Definition: Any process pertaining to the functions of the nervous and muscular systems of an organism.